flavanone 7-O-glucoside 2''-O-beta-L-rhamnosyltransferase activity [GO:0033835] (molecular function) Definition: Catalysis of the reaction: UDP-L-rhamnose + a flavanone 7-O-glucoside = UDP + a flavanone 7-O-[beta-L-rhamnosyl-(1->2)-beta-D-glucoside]. Also known as: 1->2 UDP-rhamnosyltransferase activity, UDP-L-rhamnose:flavanone-7-O-glucoside 2''-O-beta-L-rhamnosyltransferase activity, UDP-rhamnose:flavanone-7-O-glucoside-2''-O-rhamnosyltransferase activity Sources: EC:2.4.1.236 Relationships: is a type of hexosyltransferase activity [GO:0016758]